{
  "gene_name": "POZ-, AT hook-, and zinc finger-containing protein 1",
  "term_label": "nucleoplasm",
  "term_id": "GO:0005654",
  "gene": "UniProtKB:Q9HBE1",
  "gene_symbol": "PATZ1"
}